{
  "gene_name": "Putative uncharacterized protein ZNF295-AS1",
  "gene_symbol": "ZNF295-AS1",
  "gene": "UniProtKB:Q8N0V1",
  "term_label": "Unknown cellular component",
  "term_id": "UNKNOWN:0003"
}